{
  "gene_symbol": "RHOT1",
  "gene": "UniProtKB:Q8IXI2",
  "term_id": "GO:0047497",
  "term_label": "mitochondrion transport along microtubule",
  "gene_name": "Mitochondrial Rho GTPase 1"
}